positive regulation of ferulate catabolic process [GO:1901468] (biological process) Definition: Any process that activates or increases the frequency, rate or extent of ferulate catabolic process. Sources: GOC:TermGenie, GOC:mengo_curators Relationships: is a type of GO:0009896; is a type of positive regulation of small molecule metabolic process [GO:0062013]; is a type of GO:1901466; positively regulates ferulate catabolic process [GO:1901067] Also known as: activation of ferulate breakdown, activation of ferulate catabolism, activation of ferulate degradation, positive regulation of ferulate breakdown, positive regulation of ferulate catabolism, positive regulation of ferulate degradation, up regulation of ferulate breakdown, up regulation of ferulate catabolic process, up regulation of ferulate catabolism, up regulation of ferulate degradation, up-regulation of ferulate breakdown, up-regulation of ferulate catabolic process, up-regulation of ferulate catabolism, up-regulation of ferulate degradation, upregulation of ferulate breakdown, upregulation of ferulate catabolic process, upregulation of ferulate catabolism, upregulation of ferulate degradation, activation of ferulate catabolic process